rhombomere 3 development [GO:0021569] (biological process) Relationships: is a type of GO:0021546 Sources: GOC:cls, GOC:curators, GOC:dgh, GOC:dph, GOC:jid Definition: The process whose specific outcome is the progression of rhombomere 3 over time, from its formation to the mature structure. Rhombomeres are transverse segments of the developing rhombencephalon. Rhombomeres are lineage restricted, express different genes from one another, and adopt different developmental fates. Rhombomeres are numbered in anterior to posterior order.